{
  "term_label": "ubiquitin-like ligase-substrate adaptor activity",
  "gene_symbol": "ASB1",
  "gene": "UniProtKB:Q9Y576",
  "gene_name": "Ankyrin repeat and SOCS box protein 1",
  "term_id": "GO:1990756"
}